mitotic cohesin complex [GO:0030892] (cellular component) References: PMID:12750522 Sources: GOC:mah Relationships: is a type of cohesin complex [GO:0008278] Also known as: nuclear mitotic cohesin complex Definition: A cohesin complex that mediates sister chromatid cohesion during mitosis; has a subunit composition distinct from that of the meiotic cohesin complex.